{
  "gene_name": "Mediator of RNA polymerase II transcription subunit 31",
  "term_id": "GO:0070847",
  "term_label": "core mediator complex",
  "gene_symbol": "MED31",
  "gene": "UniProtKB:Q9Y3C7"
}